{
  "term_id": "GO:0045744",
  "term_label": "negative regulation of G protein-coupled receptor signaling pathway",
  "gene": "UniProtKB:Q9NS28",
  "gene_name": "Regulator of G-protein signaling 18",
  "gene_symbol": "RGS18"
}